violaceol I biosynthetic process [GO:1900590] (BP) Also known as: violaceol I anabolism, violaceol I biosynthesis, violaceol I formation, violaceol I synthesis Sources: GOC:TermGenie, GOC:di Definition: The chemical reactions and pathways resulting in the formation of violaceol I. Relationships: is a type of catechol-containing compound biosynthetic process [GO:0009713]; is a type of secondary metabolite biosynthetic process [GO:0044550]; is a type of violaceol I metabolic process [GO:1900588]; is_a ether biosynthetic process [GO:1901503] Regulation: regulated by GO:1900713; negatively regulated by negative regulation of violaceol I biosynthetic process [GO:1900714]; positively regulated by positive regulation of violaceol I biosynthetic process [GO:1900715]